intussusceptive angiogenesis [GO:0002041] (biological process) Relationships: is a type of angiogenesis [GO:0001525] References: PMID:16391003 Definition: The formation of new blood vessels as a result of the insertion and extension of lumenal tissue pillars.